{
  "gene": "UniProtKB:Q7Z2X4",
  "term_id": "GO:0005737",
  "gene_symbol": "PID1",
  "gene_name": "PTB-containing, cubilin and LRP1-interacting protein",
  "term_label": "cytoplasm"
}